central nervous system development [GO:0007417] (biological process) Sources: GOC:bf, GOC:jid, ISBN:0582227089 Relationships: is a type of system development [GO:0048731]; is part of GO:0007399 Also known as: CNS development Definition: The process whose specific outcome is the progression of the central nervous system over time, from its formation to the mature structure. The central nervous system is the core nervous system that serves an integrating and coordinating function. In vertebrates it consists of the brain and spinal cord. In those invertebrates with a central nervous system it typically consists of a brain, cerebral ganglia and a nerve cord.